{
  "term_label": "RNA polymerase II cis-regulatory region sequence-specific DNA binding",
  "gene": "UniProtKB:P15408",
  "gene_name": "Fos-related antigen 2",
  "gene_symbol": "FOSL2",
  "term_id": "GO:0000978"
}